{
  "gene": "UniProtKB:Q99590",
  "term_label": "Unknown molecular function",
  "term_id": "UNKNOWN:0001",
  "gene_symbol": "SCAF11",
  "gene_name": "Protein SCAF11"
}